postnatal olfactory bulb interneuron migration [GO:0021827] (biological process) References: PMID:12626695 Sources: GOC:cls, GOC:dgh, GOC:dph, GOC:jid, GO_REF:0000021 Relationships: is a type of cerebral cortex tangential migration using cell-cell interactions [GO:0021823]; is_a tangential migration from the subventricular zone to the olfactory bulb [GO:0022028]; is part of olfactory bulb interneuron development [GO:0021891] Definition: The migration of olfactory bulb interneuron precursors in the cerebral cortex that occurs after birth.